{
  "term_label": "Unknown biological process",
  "gene_name": "T cell receptor alpha joining 48 (Fragment)",
  "gene": "UniProtKB:A0A075B6V3",
  "gene_symbol": "TRAJ48",
  "term_id": "UNKNOWN:0002"
}